{
  "term_label": "ceramide biosynthetic process",
  "term_id": "GO:0046513",
  "gene_symbol": "SMPD1",
  "gene_name": "Sphingomyelin phosphodiesterase",
  "gene": "UniProtKB:P17405"
}